{
  "gene_symbol": "SLC25A16",
  "gene": "UniProtKB:P16260",
  "gene_name": "Solute carrier family 25 member 16",
  "term_label": "mitochondrial coenzyme A transmembrane transport",
  "term_id": "GO:1990559"
}